{
  "term_label": "transcription coactivator activity",
  "term_id": "GO:0003713",
  "gene": "UniProtKB:O75529",
  "gene_name": "TAF5-like RNA polymerase II p300_CBP-associated factor-associated factor 65 kDa subunit 5L",
  "gene_symbol": "TAF5L"
}